{
  "gene": "UniProtKB:O75592",
  "term_id": "GO:0008582",
  "gene_symbol": "MYCBP2",
  "gene_name": "E3 ubiquitin-protein ligase MYCBP2",
  "term_label": "regulation of synaptic assembly at neuromuscular junction"
}